{
  "gene_name": "Dynein axonemal intermediate chain 7",
  "term_id": "UNKNOWN:0002",
  "gene": "UniProtKB:Q6TDU7",
  "gene_symbol": "DNAI7",
  "term_label": "Unknown biological process"
}